{
  "gene": "UniProtKB:C9JSJ3",
  "term_id": "UNKNOWN:0003",
  "term_label": "Unknown cellular component",
  "gene_name": "Meiosis initiator protein",
  "gene_symbol": "MEIOSIN"
}